{
  "gene_name": "Krueppel-like factor 5",
  "term_label": "DNA-binding transcription factor activity, RNA polymerase II-specific",
  "gene_symbol": "KLF5",
  "term_id": "GO:0000981",
  "gene": "UniProtKB:Q13887"
}